{
  "gene": "UniProtKB:Q8WV16",
  "gene_symbol": "DCAF4",
  "term_id": "UNKNOWN:0002",
  "term_label": "Unknown biological process",
  "gene_name": "DDB1- and CUL4-associated factor 4"
}